{
  "gene": "UniProtKB:Q9BPU9",
  "gene_name": "B9 domain-containing protein 2",
  "term_label": "MKS complex",
  "term_id": "GO:0036038",
  "gene_symbol": "B9D2"
}